{
  "gene_symbol": "OSBPL3",
  "gene": "UniProtKB:Q9H4L5",
  "term_id": "GO:0015485",
  "gene_name": "Oxysterol-binding protein-related protein 3",
  "term_label": "cholesterol binding"
}